{
  "gene_symbol": "TNRC6A",
  "gene_name": "Trinucleotide repeat-containing gene 6A protein",
  "gene": "UniProtKB:Q8NDV7",
  "term_id": "GO:0005654",
  "term_label": "nucleoplasm"
}